{
  "term_label": "cytoplasm",
  "gene_name": "RISC-loading complex subunit TARBP2",
  "gene": "UniProtKB:Q15633",
  "term_id": "GO:0005737",
  "gene_symbol": "TARBP2"
}